{
  "gene_name": "Dehydrodolichyl diphosphate synthase complex subunit DHDDS",
  "term_id": "GO:0045547",
  "gene_symbol": "DHDDS",
  "term_label": "ditrans,polycis-polyprenyl diphosphate synthase [(2E,6E)-farnesyl diphosphate specific] activity",
  "gene": "UniProtKB:Q86SQ9"
}